{
  "gene_name": "WD repeat domain phosphoinositide-interacting protein 2",
  "term_label": "autophagy of mitochondrion",
  "term_id": "GO:0000422",
  "gene_symbol": "WIPI2",
  "gene": "UniProtKB:Q9Y4P8"
}